regulation of meiotic cell cycle [GO:0051445] (biological process) Definition: Any process that modulates the rate or extent of progression through the meiotic cell cycle. Relationships: is a type of regulation of cell cycle [GO:0051726]; is a type of GO:2000241; regulates GO:0051321 Also known as: meiotic cell cycle modulation, meiotic cell cycle regulation, modulation of meiotic cell cycle progression, regulation of meiotic cell cycle progression, regulation of progression through meiotic cell cycle, meiotic cell cycle regulator Subtypes: regulation of sexual sporulation [GO:0034306], regulation of meiotic nuclear division [GO:0040020], positive regulation of meiotic cell cycle [GO:0051446], negative regulation of meiotic cell cycle [GO:0051447], regulation of cell cycle switching, mitotic to meiotic cell cycle [GO:0110044], regulation of initiation of premeiotic DNA replication [GO:1904512] Sources: GOC:ai, GOC:dph, GOC:tb